{
  "gene_name": "GTPase HRas",
  "term_label": "GTPase activity",
  "gene_symbol": "HRAS",
  "term_id": "GO:0003924",
  "gene": "UniProtKB:P01112"
}